{
  "gene_name": "Egl nine homolog 1",
  "term_label": "cytoplasm",
  "gene_symbol": "EGLN1",
  "term_id": "GO:0005737",
  "gene": "UniProtKB:Q9GZT9"
}